{
  "gene_symbol": "KRTAP25-1",
  "term_label": "Unknown biological process",
  "term_id": "UNKNOWN:0002",
  "gene_name": "Keratin-associated protein 25-1",
  "gene": "UniProtKB:Q3LHN0"
}